glucose metabolic process [GO:0006006] (biological process) Definition: The chemical reactions and pathways involving glucose, the aldohexose gluco-hexose. D-glucose is dextrorotatory and is sometimes known as dextrose; it is an important source of energy for living organisms and is found free as well as combined in homo- and hetero-oligosaccharides and polysaccharides. Relationships: is a type of GO:0019318 Sources: ISBN:0198506732 Subtypes: glucose catabolic process [GO:0006007], gluconeogenesis [GO:0006094], sucrose catabolic process via 3'-ketosucrose [GO:0019574], poly(hydroxyalkanoate) biosynthetic process from glucose [GO:1902924] Also known as: cellular glucose metabolic process, glucose metabolism Regulation: regulated by regulation of glucose metabolic process [GO:0010906]; positively regulated by GO:0010907